negative regulation of central B cell deletion [GO:0002899] (biological process) Sources: GOC:add Definition: Any process that stops, prevents, or reduces the frequency, rate, or extent of central B cell deletion. Also known as: down regulation of central B cell deletion, down-regulation of central B cell deletion, downregulation of central B cell deletion, inhibition of central B cell deletion Relationships: is a type of negative regulation of B cell deletion [GO:0002868]; is a type of negative regulation of central B cell tolerance induction [GO:0002896]; is a type of regulation of central B cell deletion [GO:0002898]; is a type of negative regulation of B cell differentiation [GO:0045578]; negatively regulates GO:0002342